{
  "gene_name": "Interleukin-12 receptor subunit beta-2",
  "term_id": "GO:0004896",
  "term_label": "cytokine receptor activity",
  "gene_symbol": "IL12RB2",
  "gene": "UniProtKB:Q99665"
}